{
  "term_label": "receptor complex",
  "gene": "UniProtKB:P36894",
  "gene_name": "Bone morphogenetic protein receptor type-1A",
  "gene_symbol": "BMPR1A",
  "term_id": "GO:0043235"
}